{
  "gene": "UniProtKB:Q6EMK4",
  "term_label": "signaling receptor activity",
  "gene_name": "Vasorin",
  "gene_symbol": "VASN",
  "term_id": "GO:0038023"
}